{
  "gene_name": "Protein S100-A9",
  "gene": "UniProtKB:P06702",
  "term_label": "neutrophil chemotaxis",
  "gene_symbol": "S100A9",
  "term_id": "GO:0030593"
}